{
  "gene": "UniProtKB:P52799",
  "gene_name": "Ephrin-B2",
  "term_id": "GO:0042734",
  "term_label": "presynaptic membrane",
  "gene_symbol": "EFNB2"
}